glial cell fate specification [GO:0021780] (BP) Definition: The process in which a cell becomes capable of differentiating autonomously into a glial cell in an environment that is neutral with respect to the developmental pathway. Upon specification, the cell fate can be reversed. Relationships: is a type of cell fate specification [GO:0001708]; is part of glial cell fate commitment [GO:0021781] Subtypes: oligodendrocyte cell fate specification [GO:0021778] Sources: GOC:cls, GOC:dgh, GOC:dph, GOC:jid, GO_REF:0000021